{
  "gene_symbol": "ZIM3",
  "term_id": "GO:0000978",
  "term_label": "RNA polymerase II cis-regulatory region sequence-specific DNA binding",
  "gene": "UniProtKB:Q96PE6",
  "gene_name": "Zinc finger imprinted 3"
}